{
  "term_label": "external side of plasma membrane",
  "gene": "UniProtKB:O75015",
  "gene_symbol": "FCGR3B",
  "term_id": "GO:0009897",
  "gene_name": "Low affinity immunoglobulin gamma Fc region receptor III-B"
}